{
  "term_label": "plasma membrane",
  "gene_symbol": "ASIC4",
  "gene": "UniProtKB:Q96FT7",
  "term_id": "GO:0005886",
  "gene_name": "Acid-sensing ion channel 4"
}